{
  "gene_symbol": "PDSS2",
  "term_label": "isoprenoid biosynthetic process",
  "gene": "UniProtKB:Q86YH6",
  "term_id": "GO:0008299",
  "gene_name": "All trans-polyprenyl-diphosphate synthase PDSS2"
}